negative regulation of tRNA export from nucleus [GO:2000239] (biological process) Sources: GOC:mah Also known as: negative regulation of tRNA export from cell nucleus, negative regulation of tRNA export out of nucleus, negative regulation of tRNA transport from nucleus to cytoplasm, negative regulation of tRNA-nucleus export Relationships: is a type of negative regulation of RNA export from nucleus [GO:0046832]; is a type of negative regulation of ribonucleoprotein complex localization [GO:2000198]; is a type of regulation of tRNA export from nucleus [GO:2000238]; negatively regulates tRNA export from nucleus [GO:0006409] Definition: Any process that stops, prevents, or reduces the frequency, rate or extent of tRNA export from nucleus.